guanine/guanine mispair binding [GO:0035489] (molecular function) Relationships: is a type of mismatched DNA binding [GO:0030983] Also known as: G/G mispair binding Sources: GOC:bf, GOC:jh Definition: Binding to a double-stranded DNA region containing a G/G mispair.